{
  "gene": "UniProtKB:P0DMV8",
  "gene_name": "Heat shock 70 kDa protein 1A",
  "term_id": "GO:0016887",
  "term_label": "ATP hydrolysis activity",
  "gene_symbol": "HSPA1A"
}